postsynaptic neurotransmitter receptor diffusion trapping [GO:0098970] (biological process) References: PMID:18832033 Regulation: regulated by regulation of postsynaptic neurotransmitter receptor diffusion trapping [GO:0150054] Definition: The process by which diffusing neurotransmitter receptor becomes trapped at the postsynaptic specialization membrane. This is typically due to interaction with components of the post-synaptic specialization. Relationships: is a type of receptor localization to synapse [GO:0097120]; is a type of GO:0099072; is_a neurotransmitter receptor diffusion trapping [GO:0099628]; occurs in postsynaptic membrane [GO:0045211]; occurs in postsynaptic specialization membrane [GO:0099634]